{
  "term_label": "release of cytochrome c from mitochondria",
  "term_id": "GO:0001836",
  "gene_name": "Induced myeloid leukemia cell differentiation protein Mcl-1",
  "gene_symbol": "MCL1",
  "gene": "UniProtKB:Q07820"
}